{
  "term_label": "E-box binding",
  "gene_name": "Oligodendrocyte transcription factor 3",
  "term_id": "GO:0070888",
  "gene": "UniProtKB:Q7RTU3",
  "gene_symbol": "OLIG3"
}